{
  "term_id": "UNKNOWN:0003",
  "gene": "UniProtKB:Q96R09",
  "gene_symbol": "OR5B2",
  "term_label": "Unknown cellular component",
  "gene_name": "Olfactory receptor 5B2"
}